{
  "gene_symbol": "DEFA3",
  "gene_name": "Neutrophil defensin 3",
  "gene": "UniProtKB:P59666",
  "term_id": "GO:0061844",
  "term_label": "antimicrobial humoral immune response mediated by antimicrobial peptide"
}